{
  "gene_name": "Lysine-rich nucleolar protein 1",
  "term_label": "Unknown molecular function",
  "term_id": "UNKNOWN:0001",
  "gene": "UniProtKB:Q1ED39",
  "gene_symbol": "KNOP1"
}